{
  "gene_name": "5-hydroxytryptamine receptor 3E",
  "term_id": "GO:0140227",
  "gene_symbol": "HTR3E",
  "gene": "UniProtKB:A5X5Y0",
  "term_label": "serotonin-gated cation-selective signaling pathway"
}